{
  "term_id": "GO:0005179",
  "gene_symbol": "NPPA",
  "gene": "UniProtKB:P01160",
  "gene_name": "Natriuretic peptides A",
  "term_label": "hormone activity"
}